cysteine biosynthetic process from serine [GO:0006535] (biological process) Definition: The chemical reactions and pathways resulting in the formation of cysteine from other compounds, including serine. Sources: GOC:go_curators Also known as: cysteine anabolism from serine, cysteine formation from serine, cysteine synthesis from serine Relationships: is a type of L-serine metabolic process [GO:0006563]; is a type of cysteine biosynthetic process [GO:0019344]